male meiosis chromosome segregation [GO:0007060] (biological process) Definition: The cell cycle process in which genetic material, in the form of chromosomes, is organized and then physically separated and apportioned to two or more sets during the meiotic cell cycle in a male. Sources: GOC:ai Relationships: is a type of meiotic chromosome segregation [GO:0045132]; is part of male meiotic nuclear division [GO:0007140] Subtypes: male meiosis chromosome separation [GO:0051308]